{
  "term_label": "base-excision repair",
  "term_id": "GO:0006284",
  "gene_name": "DNA repair protein complementing XP-A cells",
  "gene": "UniProtKB:P23025",
  "gene_symbol": "XPA"
}